pigment granule membrane [GO:0090741] (CC) Subtypes: melanosome membrane [GO:0033162] References: PMID:11294610 Relationships: is_a GO:0030659; is_a bounding membrane of organelle [GO:0098588]; is part of pigment granule [GO:0048770] Definition: Any membrane that is part of a pigment granule.